{
  "term_id": "GO:0043025",
  "gene_name": "Neurensin-1",
  "term_label": "neuronal cell body",
  "gene": "UniProtKB:Q8IZ57",
  "gene_symbol": "NRSN1"
}